{
  "term_label": "synaptic vesicle fusion to presynaptic active zone membrane",
  "gene_name": "Synaptosomal-associated protein 47",
  "term_id": "GO:0031629",
  "gene": "UniProtKB:Q5SQN1",
  "gene_symbol": "SNAP47"
}